{
  "gene_name": "Kelch-like protein 17",
  "gene_symbol": "KLHL17",
  "term_id": "GO:0043161",
  "term_label": "proteasome-mediated ubiquitin-dependent protein catabolic process",
  "gene": "UniProtKB:Q6TDP4"
}